{
  "term_id": "GO:0007018",
  "gene_name": "Kinesin-like protein KIF3C",
  "term_label": "microtubule-based movement",
  "gene_symbol": "KIF3C",
  "gene": "UniProtKB:O14782"
}